negative regulation of regulated secretory pathway [GO:1903306] (biological process) Also known as: down regulation of regulated secretory pathway, down-regulation of regulated secretory pathway, downregulation of regulated secretory pathway, inhibition of regulated secretory pathway Definition: Any process that stops, prevents or reduces the frequency, rate or extent of regulated secretory pathway. Subtypes: GO:0043301, negative regulation of calcium ion-dependent exocytosis [GO:0045955], GO:2000301 References: PMID:12526776 Sources: GOC:PARL, GOC:TermGenie, GOC:pad, GO_REF:0000058 Note: An example of this is protein domain-specific expression of Synaptotagmin 1 in rat (P21707) in PMID:12526776 inferred from mutant phenotype. Relationships: is a type of negative regulation of exocytosis [GO:0045920]; is a type of regulation of regulated secretory pathway [GO:1903305]; negatively regulates regulated exocytosis [GO:0045055]